{
  "gene": "UniProtKB:Q86VS8",
  "term_label": "cytoplasmic microtubule organization",
  "term_id": "GO:0031122",
  "gene_name": "Protein Hook homolog 3",
  "gene_symbol": "HOOK3"
}